{
  "term_id": "GO:0032273",
  "gene_symbol": "TPPP3",
  "gene_name": "Tubulin polymerization-promoting protein family member 3",
  "term_label": "positive regulation of protein polymerization",
  "gene": "UniProtKB:Q9BW30"
}